{
  "gene": "UniProtKB:Q9Y2K3",
  "gene_symbol": "MYH15",
  "term_label": "Unknown biological process",
  "term_id": "UNKNOWN:0002",
  "gene_name": "Myosin-15"
}